positive regulation of thyroid hormone receptor signaling pathway [GO:0002157] (biological process) Definition: Any process that increases the frequency, rate or extent of thyroid hormone mediated signaling pathway. Sources: GOC:hjd Also known as: positive regulation of thyroid hormone mediated signaling pathway, positive regulation of thyroid hormone mediated signalling pathway Relationships: is a type of regulation of thyroid hormone receptor signaling pathway [GO:0002155]; is a type of GO:1902533; positively regulates thyroid hormone receptor signaling pathway [GO:0002154]